{
  "gene": "UniProtKB:Q8TCZ7",
  "gene_symbol": "LINC00308",
  "term_label": "Unknown molecular function",
  "term_id": "UNKNOWN:0001",
  "gene_name": "Putative uncharacterized protein encoded by LINC00308"
}